endothelial tube morphogenesis [GO:0061154] (BP) Definition: The process in which the anatomical structures of a tube are generated and organized from an endothelium. Endothelium refers to the layer of cells lining blood vessels, lymphatics, the heart, and serous cavities, and is derived from bone marrow or mesoderm. Corneal endothelium is a special case, derived from neural crest cells. Regulation: regulated by regulation of endothelial tube morphogenesis [GO:1901509]; negatively regulated by GO:1905955; positively regulated by positive regulation of endothelial tube morphogenesis [GO:1905956] Relationships: is a type of morphogenesis of an endothelium [GO:0003159]; is a type of epithelial tube morphogenesis [GO:0060562] Subtypes: GO:0061155, blood vessel lumenization [GO:0072554], GO:0097498 Sources: GOC:dph, GOC:yaf